positive regulation of cell septum assembly [GO:1901893] (biological process) Subtypes: positive regulation of division septum assembly [GO:0010973] Sources: GOC:TermGenie Relationships: is a type of positive regulation of cellular component biogenesis [GO:0044089]; is a type of positive regulation of cellular component organization [GO:0051130]; is_a positive regulation of cell cycle process [GO:0090068]; is a type of regulation of cell septum assembly [GO:1901891]; positively regulates cell septum assembly [GO:0090529] Also known as: up regulation of cell septum assembly, up-regulation of cell septum assembly, upregulation of cell septum assembly, activation of cell septum assembly Definition: Any process that activates or increases the frequency, rate or extent of cell septum assembly.